{
  "term_id": "GO:0030515",
  "gene_name": "U3 small nucleolar ribonucleoprotein protein IMP4",
  "gene": "UniProtKB:Q96G21",
  "term_label": "snoRNA binding",
  "gene_symbol": "IMP4"
}